{
  "gene_symbol": "PTPRJ",
  "term_id": "GO:0004725",
  "gene": "UniProtKB:Q12913",
  "gene_name": "Receptor-type tyrosine-protein phosphatase eta",
  "term_label": "protein tyrosine phosphatase activity"
}